{
  "gene_name": "Insulin-like growth factor 2 mRNA-binding protein 1",
  "term_label": "cytosol",
  "term_id": "GO:0005829",
  "gene_symbol": "IGF2BP1",
  "gene": "UniProtKB:Q9NZI8"
}